dendritic spine organization [GO:0097061] (biological process) Relationships: is a type of postsynapse organization [GO:0099173]; is a type of neuron projection organization [GO:0106027] Subtypes: dendritic spine morphogenesis [GO:0060997], dendritic spine maintenance [GO:0097062] Definition: A process that is carried out at the cellular level which results in the assembly, arrangement of constituent parts, or disassembly of a dendritic spine. A dendritic spine is a specialized protrusion from a neuronal dendrite and is involved in synaptic transmission. Also known as: dendritic spine organisation References: PMID:20410104 Sources: GOC:BHF